{
  "gene_symbol": "MPDZ",
  "gene_name": "Multiple PDZ domain protein",
  "term_id": "GO:0005737",
  "term_label": "cytoplasm",
  "gene": "UniProtKB:O75970"
}